endocytosis, site selection [GO:0120207] (biological process) Definition: The process of selecting and or marking the position where endocytosis will occur. References: PMID:30044717 Sources: GOC:vw Relationships: is a type of protein localization to cell periphery [GO:1990778]; is part of GO:0006897